{
  "gene_name": "Pleckstrin homology domain-containing family G member 4B",
  "gene_symbol": "PLEKHG4B",
  "term_label": "plasma membrane",
  "term_id": "GO:0005886",
  "gene": "UniProtKB:Q96PX9"
}